ecdysteroid 25-hydroxylase activity [GO:0035302] (molecular function) Note: Note that in the ecdysteroidogenic pathway, this activity catalyzes the conversion of 2,22,25-trideoxyecdysone (3-beta,5-beta-ketodiol) to 2,22-dideoxyecdysone (3-beta,5-beta-ketotriol). Relationships: is a type of GO:0008395; is a type of oxidoreductase activity, acting on paired donors, with incorporation or reduction of molecular oxygen, reduced flavin or flavoprotein as one donor, and incorporation of one atom of oxygen [GO:0016712] Definition: Catalysis of the hydroxylation of an ecdysteroid at carbon position 25. References: PMID:15350618